peptidyl-tyrosine dehydrogenation [GO:0018251] (biological process) Relationships: is a type of peptidyl-tyrosine modification [GO:0018212]; is a type of protein dehydration [GO:0018249] Note: See also the biological process terms 'peptide cross-linking via L-seryl-5-imidazolinone glycine ; GO:0018252' and 'peptide cross-linking via 2-imino-glutaminyl-5-imidazolinone glycine ; GO:0019729'. Sources: RESID:AA0183 Definition: The oxidation of the C alpha-C beta bond of peptidyl-tyrosine to form peptidyl-dehydrotyrosine coupled with cyclization of neighboring residues.